palmatine biosynthetic process [GO:0035831] (biological process) References: PMID:21327819 Sources: GOC:yaf Definition: The chemical reactions and pathways resulting in the formation of palmatine, a berberine alkaloid found in many plants. Relationships: is a type of isoquinoline alkaloid biosynthetic process [GO:0033075] Also known as: palmatine anabolism, palmatine biosynthesis, palmatine formation, palmatine synthesis